{
  "gene_name": "Putative protein ATXN8OS",
  "term_label": "Unknown cellular component",
  "term_id": "UNKNOWN:0003",
  "gene": "UniProtKB:P0DMR3",
  "gene_symbol": "ATXN8OS"
}